{
  "gene_symbol": "NUDT4B",
  "term_id": "GO:1901909",
  "gene": "UniProtKB:A0A024RBG1",
  "gene_name": "Diphosphoinositol polyphosphate phosphohydrolase NUDT4B",
  "term_label": "diadenosine hexaphosphate catabolic process"
}